{
  "term_id": "GO:0005543",
  "gene_symbol": "SYT16",
  "term_label": "phospholipid binding",
  "gene": "UniProtKB:Q17RD7",
  "gene_name": "Synaptotagmin-16"
}